LinE complex [GO:0062119] (cellular component) Definition: A protein complex that associates with chromatin to form linear elements in fission yeast. In S. pombe, the LinE complex contains four main structural components (Rec10, Rec25, Rec27, and Mug20) and other associated proteins. Relationships: is a type of nuclear protein-containing complex [GO:0140513] References: PMID:30640914